{
  "gene": "UniProtKB:P51159",
  "term_id": "GO:0070382",
  "gene_name": "Ras-related protein Rab-27A",
  "gene_symbol": "RAB27A",
  "term_label": "exocytic vesicle"
}